{
  "gene_symbol": "TBX5",
  "term_id": "GO:0000978",
  "gene": "UniProtKB:Q99593",
  "term_label": "RNA polymerase II cis-regulatory region sequence-specific DNA binding",
  "gene_name": "T-box transcription factor TBX5"
}